{
  "gene_symbol": "DEFB136",
  "term_id": "GO:0140367",
  "gene": "UniProtKB:Q30KP8",
  "gene_name": "Defensin beta 136",
  "term_label": "antibacterial innate immune response"
}